positive regulation of cyclodextrin catabolic process [GO:2000959] (biological process) Definition: Any process that activates or increases the frequency, rate or extent of cyclodextrin catabolic process. Sources: GOC:mengo_curators Relationships: is a type of positive regulation of catabolic process [GO:0009896]; is a type of positive regulation of macromolecule metabolic process [GO:0010604]; is a type of GO:0045913; is_a regulation of cyclodextrin catabolic process [GO:2000957]; positively regulates GO:2000901 Also known as: positive regulation of cyclodextrin catabolism